blepharoplast [GO:0097727] (cellular component) Note: The blepharoplast should not be confused with a basal body; rather, it acts as the precursor assembly zone for multiple basal bodies. Definition: An intracellular non-membrane-bounded organelle found in multi-ciliated sperm cells of some primitive land plants, and consisting of many radially arranged ninefold symmetric cylinders. The blepharoplast is involved in de novo formation of multiple centrioles; it enlarges and then disintegrates into many procentrioles, which elongate and ultimately nucleate cilia on the surface of the sperm cell. Relationships: is a type of intracellular membraneless organelle [GO:0043232] References: PMID:22691130, PMID:25047614 Sources: GOC:cilia, GOC:tb